limonoid glucosyltransferase activity [GO:0050645] (molecular function) Definition: Catalysis of the reaction: UDP-glucose + limonin = glucosyl-limonin + UDP. Relationships: is a type of GO:0035251 Also known as: LGTase activity, limonoid UDP-glucosyltransferase activity, uridine diphosphoglucose-limonoid glucosyltransferase activity Sources: EC:2.4.1.210